{
  "term_label": "Unknown molecular function",
  "term_id": "UNKNOWN:0001",
  "gene_symbol": "AMN1",
  "gene": "UniProtKB:Q8IY45",
  "gene_name": "Protein AMN1 homolog"
}